{
  "gene": "UniProtKB:P0DML2",
  "gene_name": "Chorionic somatomammotropin hormone 1",
  "term_id": "GO:0060396",
  "gene_symbol": "CSH1",
  "term_label": "growth hormone receptor signaling pathway"
}